{
  "gene": "UniProtKB:Q8NB16",
  "gene_name": "Mixed lineage kinase domain-like protein",
  "term_id": "UNKNOWN:0001",
  "term_label": "Unknown molecular function",
  "gene_symbol": "MLKL"
}